positive regulation of NK T cell activation [GO:0051135] (biological process) Definition: Any process that activates or increases the frequency, rate or extent of natural killer T cell activation. References: PMID:12154375, PMID:9133426 Sources: ISBN:0781735149 Also known as: positive regulation of NK T lymphocyte activation, positive regulation of NK T-cell activation, positive regulation of NK T-lymphocyte activation, positive regulation of NKT cell activation, positive regulation of NT cell activation, positive regulation of natural T cell activation, positive regulation of natural killer T cell activation, up regulation of NK T cell activation, up-regulation of NK T cell activation, upregulation of NK T cell activation, activation of NK T cell activation, stimulation of NK T cell activation Relationships: is a type of positive regulation of alpha-beta T cell activation [GO:0046635]; is a type of regulation of NK T cell activation [GO:0051133]; RO_0002213 NK T cell activation [GO:0051132] Subtypes: positive regulation of NK T cell proliferation [GO:0051142]